primosome complex [GO:1990077] (cellular component) Definition: Any of a family of protein complexes that form at the origin of replication or stalled replication forks and function in replication primer synthesis in all organisms. Early complexes initiate double-stranded DNA unwinding. The core unit consists of a replicative helicase and a primase. The helicase further unwinds the DNA and recruits the polymerase machinery. The primase synthesizes RNA primers that act as templates for complementary stand replication by the polymerase machinery. The primosome contains a number of associated proteins and protein complexes and contributes to the processes of replication initiation, lagging strand elongation, and replication restart. References: PMID:21856207 Sources: GOC:bhm, GOC:mah Subtypes: core primosome complex [GO:1990098], pre-primosome complex [GO:1990099], GO:1990101, GO:1990102, DnaA-HU complex [GO:1990103] Relationships: is a type of protein-DNA complex [GO:0032993]; is part of replisome [GO:0030894] Also known as: primosome